nervous system development [GO:0007399] (biological process) Regulation: regulated by regulation of nervous system development [GO:0051960]; negatively regulated by negative regulation of nervous system development [GO:0051961]; positively regulated by positive regulation of nervous system development [GO:0051962] Definition: The process whose specific outcome is the progression of nervous tissue over time, from its formation to its mature state. Relationships: is_a system development [GO:0048731] Sources: GOC:dgh Also known as: pan-neural process